{
  "gene": "UniProtKB:Q13496",
  "term_label": "negative regulation of autophagosome assembly",
  "gene_name": "Myotubularin",
  "gene_symbol": "MTM1",
  "term_id": "GO:1902902"
}